regulation of sphingolipid biosynthetic process [GO:0090153] (biological process) Relationships: is a type of regulation of macromolecule biosynthetic process [GO:0010556]; is a type of regulation of cellular component biogenesis [GO:0044087]; is a type of GO:0046890; is_a regulation of membrane lipid metabolic process [GO:1905038]; regulates sphingolipid biosynthetic process [GO:0030148] Sources: GOC:ascb_2009, GOC:dph, GOC:tb Definition: Any process that modulates the rate, frequency or extent of sphingolipid biosynthesis. Sphingolipid biosynthesis is the chemical reactions and pathways resulting in the formation of sphingolipids, any of a class of lipids containing the long-chain amine diol sphingosine or a closely related base (a sphingoid). Subtypes: positive regulation of sphingolipid biosynthetic process [GO:0090154], negative regulation of sphingolipid biosynthetic process [GO:0090155], regulation of ceramide biosynthetic process [GO:2000303]